{
  "term_id": "GO:0071578",
  "term_label": "zinc ion import across plasma membrane",
  "gene_name": "Zinc transporter ZIP6",
  "gene_symbol": "SLC39A6",
  "gene": "UniProtKB:Q13433"
}